{
  "gene": "UniProtKB:A0A0A6YYG3",
  "term_label": "plasma membrane",
  "gene_symbol": "TRBV6-8",
  "gene_name": "T cell receptor beta variable 6-8",
  "term_id": "GO:0005886"
}